{
  "term_id": "UNKNOWN:0001",
  "gene_name": "Transmembrane and coiled-coil domains protein 1",
  "gene": "UniProtKB:O94876",
  "term_label": "Unknown molecular function",
  "gene_symbol": "TMCC1"
}